{
  "gene_symbol": "TFAP2B",
  "term_label": "nucleus",
  "gene_name": "Transcription factor AP-2-beta",
  "gene": "UniProtKB:Q92481",
  "term_id": "GO:0005634"
}